{
  "term_id": "GO:0005654",
  "gene_symbol": "CHAMP1",
  "term_label": "nucleoplasm",
  "gene_name": "Chromosome alignment-maintaining phosphoprotein 1",
  "gene": "UniProtKB:Q96JM3"
}